{
  "gene": "UniProtKB:Q5K131",
  "term_label": "Unknown biological process",
  "gene_symbol": "CLLU1",
  "gene_name": "Chronic lymphocytic leukemia up-regulated protein 1",
  "term_id": "UNKNOWN:0002"
}